{
  "term_label": "Unknown cellular component",
  "term_id": "UNKNOWN:0003",
  "gene_name": "Putative uncharacterized protein CXorf42",
  "gene": "UniProtKB:Q8N9T2",
  "gene_symbol": "NKAPP1"
}